{
  "gene": "UniProtKB:P24903",
  "term_id": "GO:0020037",
  "term_label": "heme binding",
  "gene_name": "Cytochrome P450 2F1",
  "gene_symbol": "CYP2F1"
}